{
  "gene_symbol": "KIAA1958",
  "gene_name": "Uncharacterized protein KIAA1958",
  "gene": "UniProtKB:Q8N8K9",
  "term_label": "Unknown cellular component",
  "term_id": "UNKNOWN:0003"
}